effector-mediated defense to host-produced reactive oxygen species [GO:0033661] (biological process) Relationships: is_a symbiont defense to host-produced reactive oxygen species [GO:0052164] Also known as: down regulation by organism of defense-related host metabolic burst, down-regulation by organism of defense-related host oxidative burst, downregulation by organism of defense-related host AOS production, negative regulation by organism of defense-related host ROI production, negative regulation by organism of defense-related host ROS production, negative regulation by organism of defense-related host reactive oxidative species production, negative regulation by organism of defense-related host reactive oxygen intermediate production, negative regulation by organism of defense-related host respiratory burst, negative regulation by symbiont of defense-related host reactive oxygen species production, suppression by symbiont of defense-related host reactive oxygen species production Sources: GOC:pamgo_curators Definition: A process mediated by a molecule secreted by a symbiont that results in the suppression of reactive oxygen species produced by the host as part of its innate immune response. The host is defined as the larger of the organisms involved in a symbiotic interaction.